{
  "gene_symbol": "SATB1",
  "term_id": "GO:0000978",
  "gene": "UniProtKB:Q01826",
  "term_label": "RNA polymerase II cis-regulatory region sequence-specific DNA binding",
  "gene_name": "DNA-binding protein SATB1"
}